eye pigment granule organization [GO:0008057] (biological process) Definition: A process that is carried out at the cellular level which results in the assembly, arrangement of constituent parts, or disassembly of intracellular pigment storage granules in the eye. References: PMID:9303295 Also known as: eye pigment granule organisation, eye pigment granule organization and biogenesis Relationships: is a type of pigment granule organization [GO:0048753]